{
  "gene_name": "RNA-binding protein 38",
  "term_label": "mRNA 3'-UTR binding",
  "gene_symbol": "RBM38",
  "term_id": "GO:0003730",
  "gene": "UniProtKB:Q9H0Z9"
}